{
  "gene": "UniProtKB:O75054",
  "gene_name": "Immunoglobulin superfamily member 3",
  "gene_symbol": "IGSF3",
  "term_id": "GO:0016020",
  "term_label": "membrane"
}